{
  "term_id": "GO:0006955",
  "term_label": "immune response",
  "gene_name": "Probable non-functional immunoglobulin lambda variable 5-48",
  "gene": "UniProtKB:A0A075B6I7",
  "gene_symbol": "IGLV5-48"
}